urea carboxylase activity [GO:0004847] (molecular function) Definition: Catalysis of the reaction: ATP + bicarbonate + urea = ADP + 2 H+ + phosphate + urea-1-carboxylate. Sources: EC:6.3.4.6, RHEA:20896 Relationships: is a type of ligase activity, forming carbon-nitrogen bonds [GO:0016879] Also known as: ATP--urea amidolyase activity, UALase activity, UCA activity, urea amidolyase activity, urea carboxylase (hydrolysing), urea carboxylase (hydrolyzing) activity, urea:carbon-dioxide ligase (ADP-forming), urease (ATP-hydrolysing), urease (ATP-hydrolyzing) activity